{
  "gene": "UniProtKB:Q8NEZ5",
  "term_id": "UNKNOWN:0001",
  "gene_name": "F-box only protein 22",
  "gene_symbol": "FBXO22",
  "term_label": "Unknown molecular function"
}